{
  "term_label": "intracellular protein localization",
  "gene_symbol": "YWHAE",
  "gene_name": "14-3-3 protein epsilon",
  "term_id": "GO:0008104",
  "gene": "UniProtKB:P62258"
}